{
  "gene_name": "U4_U6.U5 tri-snRNP-associated protein 1",
  "term_id": "UNKNOWN:0001",
  "term_label": "Unknown molecular function",
  "gene": "UniProtKB:O43290",
  "gene_symbol": "SART1"
}